{
  "term_id": "GO:0030141",
  "gene_symbol": "SCG2",
  "gene": "UniProtKB:P13521",
  "term_label": "secretory granule",
  "gene_name": "Secretogranin-2"
}